{
  "term_id": "GO:0006400",
  "term_label": "tRNA modification",
  "gene": "UniProtKB:Q8WWH5",
  "gene_name": "Pseudouridylate synthase TRUB1",
  "gene_symbol": "TRUB1"
}